{
  "gene_name": "5'-nucleotidase domain-containing protein 4",
  "term_id": "UNKNOWN:0002",
  "gene": "UniProtKB:Q86YG4",
  "term_label": "Unknown biological process",
  "gene_symbol": "NT5DC4"
}